host cell endocytic vesicle membrane [GO:0097348] (cellular component) Definition: The lipid bilayer surrounding a host cell endocytic vesicle. Relationships: is a type of host cell cytoplasmic vesicle membrane [GO:0044162] Sources: GOC:ecd